{
  "gene_symbol": "PCDHGC5",
  "term_id": "GO:0050808",
  "gene": "UniProtKB:Q9Y5F6",
  "gene_name": "Protocadherin gamma-C5",
  "term_label": "synapse organization"
}